{
  "gene_name": "Uncharacterized protein",
  "gene": "UniProtKB:A0A1B0GW15",
  "term_id": "UNKNOWN:0002",
  "gene_symbol": "LOC122394732",
  "term_label": "Unknown biological process"
}